{
  "gene_symbol": "FBXO38",
  "gene_name": "F-box only protein 38",
  "term_label": "nucleus",
  "term_id": "GO:0005634",
  "gene": "UniProtKB:Q6PIJ6"
}